{
  "term_id": "GO:0000727",
  "term_label": "double-strand break repair via break-induced replication",
  "gene_symbol": "MCM5",
  "gene_name": "DNA replication licensing factor MCM5",
  "gene": "UniProtKB:P33992"
}